{
  "term_id": "GO:0000122",
  "gene_symbol": "CBX8",
  "gene_name": "Chromobox protein homolog 8",
  "gene": "UniProtKB:Q9HC52",
  "term_label": "negative regulation of transcription by RNA polymerase II"
}